NADH dehydrogenase complex (plastoquinone) assembly [GO:0010258] (BP) References: PMID:15608332 Definition: The aggregation, arrangement and bonding together of a set of components to form NADH:plastoquinone dehydrogenase complex, which is involved in the non-photochemical reduction of plastoquinones, as well as the cyclic electron transport around photosystem I. Relationships: is_a NADH dehydrogenase complex assembly [GO:0010257]; is a type of NAD(P)H dehydrogenase complex assembly [GO:0010275]